{
  "gene_symbol": "NHSL1",
  "term_label": "cell differentiation",
  "term_id": "GO:0030154",
  "gene": "UniProtKB:Q5SYE7",
  "gene_name": "NHS-like protein 1"
}